adhesion of symbiont spore to host [GO:0075004] (BP) Also known as: adhesion of symbiont spore to host during symbiotic interaction Sources: GOC:pamgo_curators Definition: The attachment of a spore of the symbiont to its host via adhesion molecules, general stickiness etc. The host is defined as the larger of the organisms involved in a symbiotic interaction. Relationships: is a type of GO:0044650 Note: Note that this term should not be used to annotate gene products of the host. It should only be used to annotate those gene products from the symbiont involved in this process.